{
  "term_id": "UNKNOWN:0002",
  "gene_name": "DPEP2 neighbor protein",
  "gene": "UniProtKB:A0A0U1RQF7",
  "term_label": "Unknown biological process",
  "gene_symbol": "DPEP2NB"
}